{
  "gene": "UniProtKB:P42336",
  "term_id": "GO:0043491",
  "gene_symbol": "PIK3CA",
  "term_label": "phosphatidylinositol 3-kinase/protein kinase B signal transduction",
  "gene_name": "Phosphatidylinositol 4,5-bisphosphate 3-kinase catalytic subunit alpha isoform"
}